{
  "gene_symbol": "RFX1",
  "term_id": "GO:0005634",
  "term_label": "nucleus",
  "gene": "UniProtKB:P22670",
  "gene_name": "MHC class II regulatory factor RFX1"
}